positive regulation of asexual reproduction [GO:1903666] (biological process) Definition: Any process that activates or increases the frequency, rate or extent of asexual reproduction. References: PMID:24390142 Sources: GOC:TermGenie, GO_REF:0000058 Also known as: up regulation of asexual reproduction, up-regulation of asexual reproduction, upregulation of asexual reproduction, activation of asexual reproduction Relationships: is a type of regulation of asexual reproduction [GO:1903664]; is a type of positive regulation of reproductive process [GO:2000243]; positively regulates asexual reproduction [GO:0019954] Subtypes: positive regulation of asexual sporulation resulting in formation of a cellular spore [GO:0043945], positive regulation of cell budding [GO:0045782], GO:0075307, GO:0075323